vanadium ion transmembrane transporter activity [GO:0015100] (molecular function) Relationships: is a type of transition metal ion transmembrane transporter activity [GO:0046915]; is part of GO:0015676 Sources: GOC:ai Definition: Enables the transfer of vanadium (V) ions from one side of a membrane to the other.